(R)-2-haloacid dehalogenase activity [GO:0033975] (molecular function) Also known as: 2-haloalkanoic acid dehalogenase activity, 2-haloalkanoid acid halidohydrolase activity, (R)-2-haloacid halidohydrolase activity, D-2-haloacid dehalogenase activity, D-DEX Relationships: is a type of hydrolase activity, acting on acid halide bonds, in C-halide compounds [GO:0019120] Definition: Catalysis of the reaction: (R)-2-haloacid + H2O = (S)-2-hydroxyacid + halide. Sources: EC:3.8.1.9